{
  "gene_symbol": "DEFB131A",
  "term_id": "GO:0005615",
  "gene_name": "Beta-defensin 131A",
  "gene": "UniProtKB:P59861",
  "term_label": "extracellular space"
}